{
  "gene_name": "Ret finger protein-like 2",
  "term_label": "cytoplasm",
  "gene": "UniProtKB:O75678",
  "term_id": "GO:0005737",
  "gene_symbol": "RFPL2"
}